aspartate family amino acid biosynthetic process [GO:0009067] (biological process) Relationships: is a type of L-amino acid biosynthetic process [GO:0170034]; is a type of GO:0170038 Subtypes: aspartate biosynthetic process [GO:0006532], GO:0009085, methionine biosynthetic process [GO:0009086], threonine biosynthetic process [GO:0009088], hydroxylysine biosynthetic process [GO:0046947], L-asparagine biosynthetic process [GO:0070981], GO:1901705 Also known as: aspartate family amino acid anabolism, aspartate family amino acid biosynthesis, aspartate family amino acid formation, aspartate family amino acid synthesis Definition: The chemical reactions and pathways resulting in the formation of amino acids of the aspartate family, comprising asparagine, aspartate, lysine, methionine and threonine. Sources: GOC:ai